{
  "gene": "UniProtKB:Q6UWF3",
  "term_label": "Unknown biological process",
  "gene_name": "SLP adapter and CSK-interacting membrane protein",
  "term_id": "UNKNOWN:0002",
  "gene_symbol": "SCIMP"
}